{
  "gene_name": "Probable non-functional T cell receptor beta variable 5-3",
  "term_label": "plasma membrane",
  "term_id": "GO:0005886",
  "gene_symbol": "TRBV5-3",
  "gene": "UniProtKB:A0A0A0MS03"
}